{
  "gene_symbol": "GRIN2A",
  "term_id": "GO:1904315",
  "term_label": "transmitter-gated monoatomic ion channel activity involved in regulation of postsynaptic membrane potential",
  "gene_name": "Glutamate receptor ionotropic, NMDA 2A",
  "gene": "UniProtKB:Q12879"
}